{
  "term_id": "GO:0030674",
  "gene_name": "Little elongation complex subunit 1",
  "term_label": "protein-macromolecule adaptor activity",
  "gene": "UniProtKB:Q9Y2F5",
  "gene_symbol": "ICE1"
}